{
  "term_label": "Unknown molecular function",
  "gene_name": "Shugoshin 1",
  "term_id": "UNKNOWN:0001",
  "gene_symbol": "SGO1",
  "gene": "UniProtKB:Q5FBB7"
}